{
  "term_label": "Unknown molecular function",
  "gene": "UniProtKB:Q13753",
  "gene_symbol": "LAMC2",
  "gene_name": "Laminin subunit gamma-2",
  "term_id": "UNKNOWN:0001"
}